{
  "gene_symbol": "C8B",
  "term_id": "GO:0005579",
  "gene": "UniProtKB:P07358",
  "gene_name": "Complement component C8 beta chain",
  "term_label": "membrane attack complex"
}